negative regulation of acetylcholine secretion, neurotransmission [GO:0014058] (biological process) Also known as: down regulation of acetylcholine secretion, down-regulation of acetylcholine secretion, downregulation of acetylcholine secretion, inhibition of acetylcholine secretion Definition: Any process that stops, prevents, or reduces the frequency, rate or extent of the regulated release of acetylcholine. Sources: GOC:ef Relationships: is a type of regulation of acetylcholine secretion, neurotransmission [GO:0014056]; is a type of negative regulation of synaptic transmission, cholinergic [GO:0032223]; is a type of negative regulation of neurotransmitter secretion [GO:0046929]; is a type of negative regulation of amine transport [GO:0051953]; negatively regulates GO:0014055